selenite reductase (NADPH) activity [GO:0098623] (molecular function) References: PMID:1321713 Also known as: selenite reductase activity Definition: Catalysis of the reaction: SeO3(2-) + 3 NADPH + 5H+ = H2Se +  3NADP+ + 3H2O. Relationships: is a type of oxidoreductase activity, acting on NAD(P)H [GO:0016651]